{
  "gene": "UniProtKB:P31277",
  "term_label": "embryonic skeletal joint morphogenesis",
  "gene_name": "Homeobox protein Hox-D11",
  "gene_symbol": "HOXD11",
  "term_id": "GO:0060272"
}